{
  "term_id": "GO:0044666",
  "gene": "UniProtKB:O14607",
  "gene_symbol": "UTY",
  "gene_name": "Histone demethylase UTY",
  "term_label": "MLL3/4 complex"
}